response to propan-1-ol [GO:1901427] (biological process) Definition: Any process that results in a change in state or activity of a cell or an organism (in terms of movement, secretion, enzyme production, gene expression, etc.) as a result of a propan-1-ol stimulus. Sources: GOC:TermGenie, GOC:mengo_curators Relationships: is a type of response to lipid [GO:0033993]; is a type of response to alcohol [GO:0097305] Regulation: regulated by regulation of response to propan-1-ol [GO:1901445]; negatively regulated by negative regulation of response to propan-1-ol [GO:1901446]; positively regulated by positive regulation of response to propan-1-ol [GO:1901447]